{
  "term_label": "ceramide biosynthetic process",
  "term_id": "GO:0046513",
  "gene_name": "Sphingomyelin phosphodiesterase 2",
  "gene": "UniProtKB:O60906",
  "gene_symbol": "SMPD2"
}